{
  "term_label": "regulation of DNA-templated transcription",
  "gene_name": "Zinc finger protein 341",
  "term_id": "GO:0006355",
  "gene_symbol": "ZNF341",
  "gene": "UniProtKB:Q9BYN7"
}